{
  "term_label": "Unknown cellular component",
  "term_id": "UNKNOWN:0003",
  "gene": "UniProtKB:Q9BZR8",
  "gene_name": "Apoptosis facilitator Bcl-2-like protein 14",
  "gene_symbol": "BCL2L14"
}